{
  "gene_symbol": "NEK11",
  "term_id": "GO:0004674",
  "gene_name": "Serine_threonine-protein kinase Nek11",
  "gene": "UniProtKB:Q8NG66",
  "term_label": "protein serine/threonine kinase activity"
}